{
  "gene": "UniProtKB:A0A1W2PQD8",
  "gene_name": "RNA polymerase II subunit A C-terminal domain phosphatase SSU72 like protein 2",
  "term_label": "mRNA cleavage and polyadenylation specificity factor complex",
  "term_id": "GO:0005847",
  "gene_symbol": "SSU72L2"
}